{
  "gene_name": "Catenin beta-1",
  "gene_symbol": "CTNNB1",
  "term_id": "GO:0098609",
  "gene": "UniProtKB:P35222",
  "term_label": "cell-cell adhesion"
}